{
  "term_label": "Unknown biological process",
  "term_id": "UNKNOWN:0002",
  "gene_symbol": "PPP1R36",
  "gene_name": "Protein phosphatase 1 regulatory subunit 36",
  "gene": "UniProtKB:Q96LQ0"
}